{
  "gene": "UniProtKB:Q9UKI2",
  "term_label": "plasma membrane",
  "gene_name": "Cdc42 effector protein 3",
  "gene_symbol": "CDC42EP3",
  "term_id": "GO:0005886"
}